{
  "gene_name": "BLOC-1-related complex subunit 8",
  "term_id": "UNKNOWN:0002",
  "gene": "UniProtKB:Q96FH0",
  "term_label": "Unknown biological process",
  "gene_symbol": "BORCS8"
}